{
  "term_id": "UNKNOWN:0001",
  "gene_name": "Progesterone-induced-blocking factor 1",
  "gene_symbol": "PIBF1",
  "gene": "UniProtKB:Q8WXW3",
  "term_label": "Unknown molecular function"
}